{
  "term_id": "GO:0005739",
  "gene_name": "Bifunctional methylenetetrahydrofolate dehydrogenase_cyclohydrolase 2, mitochondrial",
  "gene": "UniProtKB:Q9H903",
  "term_label": "mitochondrion",
  "gene_symbol": "MTHFD2L"
}